{
  "term_label": "acrosomal vesicle",
  "gene_name": "IQ domain-containing protein F1",
  "term_id": "GO:0001669",
  "gene_symbol": "IQCF1",
  "gene": "UniProtKB:Q8N6M8"
}